positive regulation of gliotoxin biosynthetic process [GO:1900691] (biological process) Sources: GOC:TermGenie, GOC:di Definition: Any process that activates or increases the frequency, rate or extent of gliotoxin biosynthetic process. Also known as: activation of gliotoxin anabolism, activation of gliotoxin biosynthesis, activation of gliotoxin formation, activation of gliotoxin synthesis, positive regulation of gliotoxin anabolism, positive regulation of gliotoxin biosynthesis, positive regulation of gliotoxin formation, positive regulation of gliotoxin synthesis, up regulation of gliotoxin anabolism, up regulation of gliotoxin biosynthesis, up regulation of gliotoxin biosynthetic process, up regulation of gliotoxin formation, up regulation of gliotoxin synthesis, up-regulation of gliotoxin anabolism, up-regulation of gliotoxin biosynthesis, up-regulation of gliotoxin biosynthetic process, up-regulation of gliotoxin formation, up-regulation of gliotoxin synthesis, upregulation of gliotoxin anabolism, upregulation of gliotoxin biosynthesis, upregulation of gliotoxin biosynthetic process, upregulation of gliotoxin formation, upregulation of gliotoxin synthesis, activation of gliotoxin biosynthetic process Relationships: is a type of positive regulation of amide metabolic process [GO:0034250]; is a type of GO:1900378; is a type of regulation of gliotoxin biosynthetic process [GO:1900689]; positively regulates GO:2001310